{
  "term_id": "GO:0099151",
  "gene_symbol": "LRFN4",
  "term_label": "regulation of postsynaptic density assembly",
  "gene": "UniProtKB:Q6PJG9",
  "gene_name": "Leucine-rich repeat and fibronectin type-III domain-containing protein 4"
}